{
  "gene_symbol": "CDH3",
  "gene_name": "Cadherin-3",
  "gene": "UniProtKB:P22223",
  "term_id": "GO:0008013",
  "term_label": "beta-catenin binding"
}